{
  "gene_symbol": "CRP",
  "gene_name": "C-reactive protein",
  "term_id": "GO:0001849",
  "gene": "UniProtKB:P02741",
  "term_label": "complement component C1q complex binding"
}